glucosylglycerate phosphorylase activity [GO:0110068] (molecular function) Definition: Catalysis of the reaction: glucosylglycerate + phosphate = glucose-1-phosphate + D-glycerate. Relationships: is a type of GO:0004645 References: PMID:28754708 Sources: GOC:imk